positive regulation of respiratory gaseous exchange [GO:1903942] (biological process) Definition: Any process that activates or increases the frequency, rate or extent of respiratory gaseous exchange. Relationships: is_a GO:0043576; is a type of GO:0051240; positively regulates respiratory gaseous exchange by respiratory system [GO:0007585] References: PMID:22819705 Sources: GOC:TermGenie, GO_REF:0000058 Also known as: up regulation of respiratory gaseous exchange, up-regulation of respiratory gaseous exchange, upregulation of respiratory gaseous exchange, activation of respiratory gaseous exchange